{
  "term_label": "signal transduction",
  "gene_symbol": "CASKIN2",
  "gene": "UniProtKB:Q8WXE0",
  "term_id": "GO:0007165",
  "gene_name": "Caskin-2"
}